{
  "term_label": "phospholipase inhibitor activity",
  "term_id": "GO:0004859",
  "gene": "UniProtKB:P02654",
  "gene_symbol": "APOC1",
  "gene_name": "Apolipoprotein C-I"
}